response to DNA replication checkpoint signaling [GO:0072438] (biological process) Subtypes: response to meiotic DNA replication checkpoint signaling [GO:0072441], response to mitotic DNA replication checkpoint signaling [GO:0072444] Definition: A process that occurs in response to signals generated as a result of DNA replication checkpoint signaling. Also known as: DNA replication checkpoint effector process, response to signal involved in DNA replication checkpoint Relationships: is a type of response to DNA integrity checkpoint signaling [GO:0072402] Sources: GOC:mtg_cell_cycle